{
  "gene": "UniProtKB:Q96MF0",
  "term_label": "Unknown molecular function",
  "term_id": "UNKNOWN:0001",
  "gene_symbol": "Q96MF0",
  "gene_name": "Putative uncharacterized protein LOC100506887"
}